{
  "gene_symbol": "UNQ6493_PRO21345",
  "gene_name": "Putative uncharacterized protein UNQ6493_PRO21345",
  "gene": "UniProtKB:Q6UXR8",
  "term_label": "Unknown biological process",
  "term_id": "UNKNOWN:0002"
}